{
  "gene_name": "Tubulin beta-3 chain",
  "term_id": "GO:0000278",
  "gene": "UniProtKB:Q13509",
  "gene_symbol": "TUBB3",
  "term_label": "mitotic cell cycle"
}